{
  "term_label": "elongator holoenzyme complex",
  "term_id": "GO:0033588",
  "gene_symbol": "ELP1",
  "gene": "UniProtKB:O95163",
  "gene_name": "Elongator complex protein 1"
}